phagosome maturation [GO:0090382] (BP) Subtypes: GO:0090386 Definition: A process that is carried out at the cellular level which results in the arrangement of constituent parts of a phagosome within a cell. Phagosome maturation begins with endocytosis and formation of the early phagosome and ends with the formation of the hybrid organelle, the phagolysosome. Sources: GOC:kmv, GOC:tb Regulation: regulated by GO:1905162; negatively regulated by GO:1905163; positively regulated by positive regulation of phagosome maturation [GO:1905164] Relationships: is a type of organelle organization [GO:0006996]; has part GO:0001845; has part exocytosis [GO:0006887]